{
  "gene": "UniProtKB:Q9H9J2",
  "term_id": "GO:0070125",
  "gene_symbol": "MRPL44",
  "gene_name": "Large ribosomal subunit protein mL44",
  "term_label": "mitochondrial translational elongation"
}